{
  "term_id": "GO:0005245",
  "gene": "UniProtKB:P54289",
  "gene_name": "Voltage-dependent calcium channel subunit alpha-2_delta-1",
  "term_label": "voltage-gated calcium channel activity",
  "gene_symbol": "CACNA2D1"
}